{
  "term_id": "GO:0003700",
  "gene_symbol": "ZNF660",
  "gene": "UniProtKB:Q6AZW8",
  "term_label": "DNA-binding transcription factor activity",
  "gene_name": "Zinc finger protein 660"
}